{
  "term_id": "UNKNOWN:0002",
  "gene": "UniProtKB:A0A075B6V9",
  "term_label": "Unknown biological process",
  "gene_name": "T cell receptor alpha joining 59 (non-functional) (Fragment)",
  "gene_symbol": "TRAJ59"
}